{
  "term_id": "UNKNOWN:0001",
  "term_label": "Unknown molecular function",
  "gene": "UniProtKB:Q99638",
  "gene_symbol": "RAD9A",
  "gene_name": "Cell cycle checkpoint control protein RAD9A"
}